far-red light photoreceptor activity [GO:0031516] (MF) Relationships: is a type of red or far-red light photoreceptor activity [GO:0009883]; is part of far-red light signaling pathway [GO:0010018] Sources: GOC:nln Definition: The function of absorbing and responding to electromagnetic radiation with a wavelength of approximately 730nm. The response may involve a change in conformation.